{
  "gene_symbol": "SYT1",
  "gene": "UniProtKB:P21579",
  "term_label": "regulation of synaptic vesicle exocytosis",
  "gene_name": "Synaptotagmin-1",
  "term_id": "GO:2000300"
}